{
  "gene_symbol": "ADPRM",
  "gene_name": "Manganese-dependent ADP-ribose_CDP-alcohol diphosphatase",
  "gene": "UniProtKB:Q3LIE5",
  "term_id": "GO:0008663",
  "term_label": "2',3'-cyclic-nucleotide 2'-phosphodiesterase activity"
}